{
  "gene": "UniProtKB:Q9UN70",
  "gene_symbol": "PCDHGC3",
  "term_id": "GO:0050839",
  "gene_name": "Protocadherin gamma-C3",
  "term_label": "cell adhesion molecule binding"
}